{
  "gene": "UniProtKB:A0A140TA67",
  "gene_symbol": "KRTAP9-6",
  "term_id": "UNKNOWN:0001",
  "gene_name": "Keratin-associated protein 9-6",
  "term_label": "Unknown molecular function"
}